{
  "gene": "UniProtKB:P43121",
  "gene_name": "Cell surface glycoprotein MUC18",
  "gene_symbol": "MCAM",
  "term_id": "GO:0007155",
  "term_label": "cell adhesion"
}